mating pheromone secretion involved in regulation of conjugation with cellular fusion [GO:0071835] (biological process) Relationships: is a type of mating pheromone secretion [GO:0071834]; BFO_0000050 conjugation with cellular fusion [GO:0000747] Sources: GOC:elh, GOC:jh, GOC:mah Also known as: peptide pheromone export involved in regulation of conjugation, mating-type pheromone secretion involved in conjugation, mating pheromone secretion involved in regulation of conjugation Definition: The regulated release of a mating pheromone, a peptide hormone that induces a behavioral or physiological response(s) from a responding organism or cell, that regulates the union or introduction of genetic information from compatible mating types that results in a genetically different individual. Conjugation requires direct cellular contact between the organisms.